{
  "gene": "UniProtKB:Q15428",
  "gene_name": "Splicing factor 3A subunit 2",
  "gene_symbol": "SF3A2",
  "term_id": "UNKNOWN:0001",
  "term_label": "Unknown molecular function"
}